regulation of mitotic recombination [GO:0000019] (biological process) Definition: Any process that modulates the frequency, rate or extent of DNA recombination during mitosis. Sources: GOC:go_curators Also known as: regulation of recombination within rDNA repeats Relationships: is a type of regulation of DNA recombination [GO:0000018]; regulates mitotic recombination [GO:0006312] Subtypes: GO:0032207, negative regulation of mitotic recombination [GO:0045950], GO:0045951